{
  "gene_name": "Kinesin-like protein KIF21A",
  "gene_symbol": "KIF21A",
  "gene": "UniProtKB:Q7Z4S6",
  "term_label": "microtubule binding",
  "term_id": "GO:0008017"
}